{
  "gene": "UniProtKB:O95279",
  "gene_symbol": "KCNK5",
  "term_id": "GO:0005886",
  "term_label": "plasma membrane",
  "gene_name": "Potassium channel subfamily K member 5"
}